{
  "term_label": "plasma membrane",
  "gene_symbol": "DGKA",
  "gene": "UniProtKB:P23743",
  "gene_name": "Diacylglycerol kinase alpha",
  "term_id": "GO:0005886"
}